negative regulation of neural precursor cell proliferation [GO:2000178] (biological process) Relationships: is a type of negative regulation of cell population proliferation [GO:0008285]; is a type of regulation of neural precursor cell proliferation [GO:2000177]; negatively regulates neural precursor cell proliferation [GO:0061351] Subtypes: negative regulation of neuroblast proliferation [GO:0007406], negative regulation of cerebellar granule cell precursor proliferation [GO:0021941], negative regulation of oligodendrocyte progenitor proliferation [GO:0070446], negative regulation of cell proliferation in dorsal spinal cord [GO:1902832], negative regulation of cell proliferation in midbrain [GO:1904934] Sources: GOC:dph, GOC:yaf Definition: Any process that stops, prevents, or reduces the frequency, rate or extent of neural precursor cell proliferation.